{
  "gene_symbol": "ZCCHC18",
  "term_label": "Unknown biological process",
  "gene_name": "Zinc finger CCHC domain-containing protein 18",
  "gene": "UniProtKB:P0CG32",
  "term_id": "UNKNOWN:0002"
}